{
  "term_id": "GO:0005829",
  "gene_name": "Phosphatidate phosphatase LPIN2",
  "gene_symbol": "LPIN2",
  "term_label": "cytosol",
  "gene": "UniProtKB:Q92539"
}